{
  "term_id": "GO:0046488",
  "gene_name": "Inactive phospholipase C-like protein 2",
  "term_label": "phosphatidylinositol metabolic process",
  "gene_symbol": "PLCL2",
  "gene": "UniProtKB:Q9UPR0"
}